histone H3K18ub reader activity [GO:0140254] (molecular function) Relationships: is a type of histone H3 reader activity [GO:0140006] Note: Comment: Note that the residue position corresponds to the canonical human H3 histone (UniProtKB:P84243); this residue is conserved across all eukaryotes. Residue 1 is the first residue following removal of the initiating Methionine (Met). Note that each histone is encoded by multiple genes, and sequences may vary across different genes within an organism. Definition: A histone reader that recognizes a histone H3 ubiquitinated at lysine 18. Also known as: H3K18ub modified histone binding References: PMID:29053958